negative regulation of endoplasmic reticulum calcium ion concentration [GO:0032471] (biological process) Sources: GOC:mah Subtypes: negative regulation of smooth endoplasmic reticulum calcium ion concentration [GO:0051565] Also known as: ER calcium ion concentration reduction, endoplasmic reticulum calcium ion concentration reduction, reduction of ER calcium ion concentration, reduction of calcium ion concentration in ER, reduction of calcium ion concentration in endoplasmic reticulum, reduction of endoplasmic reticulum calcium ion concentration Relationships: is_a GO:0032469 Definition: Any process that decreases the concentration of calcium ions in the endoplasmic reticulum.